{
  "term_label": "canonical Wnt signaling pathway",
  "gene_name": "Secreted frizzled-related protein 5",
  "gene_symbol": "SFRP5",
  "term_id": "GO:0060070",
  "gene": "UniProtKB:Q5T4F7"
}